{
  "gene": "UniProtKB:Q7Z6V5",
  "gene_symbol": "ADAT2",
  "term_label": "Unknown cellular component",
  "term_id": "UNKNOWN:0003",
  "gene_name": "tRNA-specific adenosine deaminase 2"
}